{
  "gene": "UniProtKB:P00325",
  "gene_name": "All-trans-retinol dehydrogenase [NAD(+)] ADH1B",
  "term_label": "retinoic acid metabolic process",
  "gene_symbol": "ADH1B",
  "term_id": "GO:0042573"
}